{
  "term_label": "late endosome membrane",
  "gene_symbol": "SPAAR",
  "gene_name": "Small regulatory polypeptide of amino acid response",
  "term_id": "GO:0031902",
  "gene": "UniProtKB:A0A1B0GVQ0"
}